{
  "term_id": "GO:0051897",
  "gene": "UniProtKB:Q16620",
  "gene_name": "BDNF_NT-3 growth factors receptor",
  "gene_symbol": "NTRK2",
  "term_label": "positive regulation of phosphatidylinositol 3-kinase/protein kinase B signal transduction"
}